arginyl-tRNA--protein transferase activity [GO:0004057] (molecular function) Relationships: is a type of aminoacyltransferase activity [GO:0016755]; is a type of GO:0140096; is a type of catalytic activity, acting on a tRNA [GO:0140101] Also known as: arginine transferase activity, arginyltransferase activity, arginyl-tRNA protein transferase activity References: PMID:16492767, PMID:9858543 Sources: RHEA:10208 Definition: Catalysis of the reaction: an N-terminal L-alpha-aminoacyl-[protein] + L-arginyl-tRNA(Arg) = H+ + N-terminal L-arginyl-L-amino acid-[protein] + tRNA(Arg).